{
  "term_label": "cilium assembly",
  "gene": "UniProtKB:Q8TDR0",
  "gene_name": "TRAF3-interacting protein 1",
  "gene_symbol": "TRAF3IP1",
  "term_id": "GO:0060271"
}